6-deoxy-6-sulfofructose-1-phosphate aldolase activity [GO:0061595] (molecular function) Definition: Catalysis of the reaction 6-deoxy-6-sulfofructose-1-phosphate = 3-sulfolactaldehyde + dihydroxyacetone phosphate. References: PMID:24463506 Relationships: is a type of GO:0016832